pyruvate biosynthetic process [GO:0042866] (biological process) Relationships: is a type of GO:0006090; is a type of monocarboxylic acid biosynthetic process [GO:0072330] Definition: The chemical reactions and pathways resulting in the formation of pyruvate, 2-oxopropanoate. Sources: GOC:go_curators Subtypes: pyruvate biosynthetic process from acetate [GO:0019687] Also known as: pyruvate anabolism, pyruvate biosynthesis, pyruvate formation, pyruvate synthesis